regulation of cell-substrate junction organization [GO:0150116] (biological process) Relationships: is a type of regulation of cellular component organization [GO:0051128]; regulates cell-substrate junction organization [GO:0150115] Definition: Any process that modulates the frequency, rate or extent of cell-substrate junction organization. Subtypes: regulation of cell-substrate junction assembly [GO:0090109], regulation of focal adhesion disassembly [GO:0120182], positive regulation of cell-substrate junction organization [GO:0150117], negative regulation of cell-substrate junction organization [GO:0150118] Sources: GOC:aruk